{
  "gene_symbol": "ZBTB22",
  "term_label": "regulation of transcription by RNA polymerase II",
  "gene": "UniProtKB:O15209",
  "gene_name": "Zinc finger and BTB domain-containing protein 22",
  "term_id": "GO:0006357"
}